bounding membrane of organelle [GO:0098588] (cellular component) Definition: The lipid bilayer that forms the outer-most layer of an organelle. Sources: GOC:dos Note: Examples include the outer membranes of double membrane bound organelles such as mitochondria as well as the bounding membranes of single-membrane bound organelles such as lysosomes. Relationships: is a type of organelle membrane [GO:0031090] Subtypes: Golgi membrane [GO:0000139], GO:0005774, GO:0010008, transport vesicle membrane [GO:0030658], Golgi-associated vesicle membrane [GO:0030660], GO:0030661, GO:0030662, GO:0030666, secretory granule membrane [GO:0030667], GO:0030867, smooth endoplasmic reticulum membrane [GO:0030868], platelet dense tubular network membrane [GO:0031095], microbody membrane [GO:0031903], organelle outer membrane [GO:0031968], aleurone grain membrane [GO:0032578], sarcoplasmic reticulum membrane [GO:0033017], acidocalcisome membrane [GO:0033102], GO:0033106, attachment organelle membrane [GO:0033111], GO:0033116, esterosome membrane [GO:0033118], microneme membrane [GO:0033163], hydrogenosomal membrane [GO:0046859], ciliary membrane [GO:0060170], pigment granule membrane [GO:0090741], multivesicular body, internal vesicle membrane [GO:0097488], GO:0098897, omegasome membrane [GO:1903349]